{
  "gene_name": "Serologically defined colon cancer antigen 8",
  "gene": "UniProtKB:Q86SQ7",
  "gene_symbol": "SDCCAG8",
  "term_id": "GO:0005813",
  "term_label": "centrosome"
}